negative regulation of phagocytosis, engulfment [GO:0060101] (biological process) Relationships: is a type of negative regulation of phagocytosis [GO:0050765]; is a type of GO:0060099; is_a negative regulation of membrane invagination [GO:1905154]; RO_0002212 phagocytosis, engulfment [GO:0006911] Subtypes: negative regulation of engulfment of apoptotic cell [GO:1901075] Definition: Any process that stops, prevents, or reduces the frequency, rate or extent of the internalization of bacteria, immune complexes and other particulate matter or of an apoptotic cell by phagocytosis. Sources: GOC:dph